{
  "term_label": "oxalate transmembrane transporter activity",
  "gene_symbol": "SLC26A8",
  "term_id": "GO:0019531",
  "gene_name": "Testis anion transporter 1",
  "gene": "UniProtKB:Q96RN1"
}